phosphatidylinositol-3,4-bisphosphate binding [GO:0043325] (molecular function) Sources: GOC:bf, GOC:go_curators Relationships: is_a GO:0043168 Definition: Binding to phosphatidylinositol-3,4-bisphosphate, a derivative of phosphatidylinositol in which the inositol ring is phosphorylated at the 3' and 4' positions.